{
  "term_label": "signal transduction",
  "gene_symbol": "PTPRH",
  "term_id": "GO:0007165",
  "gene": "UniProtKB:Q9HD43",
  "gene_name": "Receptor-type tyrosine-protein phosphatase H"
}